{
  "term_id": "GO:0001756",
  "term_label": "somitogenesis",
  "gene_name": "T-box transcription factor T",
  "gene": "UniProtKB:O15178",
  "gene_symbol": "TBXT"
}